intraciliary retrograde transport [GO:0035721] (biological process) Definition: The directed movement of large protein complexes along microtubules from the tip of a cilium (also called flagellum) toward the cell body, mediated by motor proteins. Regulation: regulated by regulation of intraciliary retrograde transport [GO:1905799]; negatively regulated by negative regulation of intraciliary retrograde transport [GO:1905800]; positively regulated by positive regulation of intraciliary retrograde transport [GO:1905801] Relationships: is a type of intraciliary transport [GO:0042073] Sources: GOC:BHF, GOC:cilia Note: Note that we deem cilium and microtubule-based flagellum to be equivalent. Also known as: intraflagellar retrograde transport